{
  "gene_symbol": "TRPV2",
  "term_id": "GO:0005886",
  "gene_name": "Transient receptor potential cation channel subfamily V member 2",
  "gene": "UniProtKB:Q9Y5S1",
  "term_label": "plasma membrane"
}